{
  "gene_name": "Osteoclast-stimulating factor 1",
  "term_label": "signal transduction",
  "gene_symbol": "OSTF1",
  "term_id": "GO:0007165",
  "gene": "UniProtKB:Q92882"
}